{
  "gene": "UniProtKB:Q8TBC5",
  "gene_symbol": "ZSCAN18",
  "term_label": "RNA polymerase II cis-regulatory region sequence-specific DNA binding",
  "term_id": "GO:0000978",
  "gene_name": "Zinc finger and SCAN domain-containing protein 18"
}